C-C chemokine receptor CCR7 signaling pathway [GO:0038118] (biological process) Relationships: is a type of chemokine-mediated signaling pathway [GO:0070098] Regulation: regulated by regulation of C-C chemokine receptor CCR7 signaling pathway [GO:1903080]; negatively regulated by negative regulation of C-C chemokine receptor CCR7 signaling pathway [GO:1903081]; positively regulated by GO:1903082 Definition: The series of molecular signals initiated by a the C-C chemokine type 7 receptor on the surface of a cell binding to one of it's physiological ligands, and ending with the regulation of a downstream cellular process, e.g. transcription. Note: This term was created to show the binding of cytokines to multiple receptor types, and vice-versa. Known agonists of chemokine receptor type 7 (CCR7) are C-C chemokines CCL19 and CCL21. Consider instead annotating to one of the child terms 'CCL19-activated CCR7 signaling pathway ; GO:0038119' and/or 'CCL21-activated CCR7 signaling pathway ; GO:0038120'. Subtypes: GO:0038119, CCL21-activated CCR7 signaling pathway [GO:0038120] Also known as: C-C chemokine receptor CCR7 signalling pathway, CCR7 signaling pathway References: PMID:15059845, PMID:15778365 Sources: GOC:signaling